{
  "term_label": "extracellular space",
  "gene_symbol": "PTH",
  "term_id": "GO:0005615",
  "gene": "UniProtKB:P01270",
  "gene_name": "Parathyroid hormone"
}